{
  "gene_name": "Somatotropin",
  "term_id": "GO:0008083",
  "gene_symbol": "GH1",
  "gene": "UniProtKB:P01241",
  "term_label": "growth factor activity"
}